L-arabinose catabolic process to D-xylulose 5-phosphate [GO:0019569] (biological process) Also known as: L-arabinose breakdown to xylulose 5-phosphate, L-arabinose degradation to xylulose 5-phosphate Relationships: is a type of L-arabinose catabolic process [GO:0019572]; is a type of D-xylulose 5-phosphate metabolic process [GO:0051167] Definition: The chemical reactions and pathways resulting in the breakdown of L-arabinose into D-xylulose 5-phosphate. Sources: GOC:go_curators